{
  "term_label": "plasma membrane",
  "gene_name": "Krev interaction trapped protein 1",
  "gene": "UniProtKB:O00522",
  "term_id": "GO:0005886",
  "gene_symbol": "KRIT1"
}